{
  "gene": "UniProtKB:Q86UU1",
  "gene_name": "Pleckstrin homology-like domain family B member 1",
  "gene_symbol": "PHLDB1",
  "term_id": "UNKNOWN:0001",
  "term_label": "Unknown molecular function"
}